{
  "gene": "UniProtKB:P09912",
  "term_label": "mitochondrial membrane",
  "gene_symbol": "IFI6",
  "term_id": "GO:0031966",
  "gene_name": "Interferon alpha-inducible protein 6"
}